{
  "term_id": "GO:0061630",
  "gene_symbol": "MSL2",
  "gene_name": "E3 ubiquitin-protein ligase MSL2",
  "gene": "UniProtKB:Q9HCI7",
  "term_label": "ubiquitin protein ligase activity"
}